{
  "gene": "UniProtKB:A6NMU1",
  "term_label": "Unknown biological process",
  "gene_name": "Olfactory receptor 52A4",
  "gene_symbol": "OR52A4P",
  "term_id": "UNKNOWN:0002"
}